{
  "term_id": "GO:0042420",
  "term_label": "dopamine catabolic process",
  "gene_symbol": "MOXD2P",
  "gene_name": "Putative DBH-like monooxygenase protein 2",
  "gene": "UniProtKB:A6NHM9"
}